regulation of ceramide biosynthetic process [GO:2000303] (biological process) Definition: Any process that modulates the frequency, rate or extent of a ceramide biosynthetic process. Sources: GOC:dph Also known as: regulation of ceramide anabolism, regulation of ceramide biosynthesis, regulation of ceramide formation, regulation of ceramide synthesis Relationships: is a type of GO:0034248; is a type of regulation of sphingolipid biosynthetic process [GO:0090153]; regulates ceramide biosynthetic process [GO:0046513] Subtypes: regulation of glucosylceramide biosynthetic process [GO:0046317], negative regulation of ceramide biosynthetic process [GO:1900060], positive regulation of ceramide biosynthetic process [GO:2000304]